regulation of inositol phosphate biosynthetic process [GO:0010919] (biological process) Subtypes: negative regulation of inositol phosphate biosynthetic process [GO:0010920], regulation of inositol trisphosphate biosynthetic process [GO:0032960], GO:0060732 Sources: GOC:BHF, GOC:dph, GOC:tb Also known as: regulation of inositol phosphate biosynthesis Definition: Any process that modulates the rate, frequency or extent of inositol phosphate biosynthesis. Inositol phosphate biosynthetic processes are the chemical reactions and pathways resulting in the formation of an inositol phosphate, 1,2,3,4,5,6-cyclohexanehexol, with one or more phosphate groups attached. Relationships: is a type of regulation of carbohydrate biosynthetic process [GO:0043255]; is a type of regulation of phosphorus metabolic process [GO:0051174]; is a type of regulation of alcohol biosynthetic process [GO:1902930]; regulates inositol phosphate biosynthetic process [GO:0032958]